{
  "gene_name": "Interleukin-27 subunit beta",
  "gene_symbol": "EBI3",
  "gene": "UniProtKB:Q14213",
  "term_label": "T cell proliferation",
  "term_id": "GO:0042098"
}